{
  "term_label": "putrescine biosynthetic process from arginine, via ornithine",
  "gene_symbol": "AZIN2",
  "gene": "UniProtKB:Q96A70",
  "gene_name": "Antizyme inhibitor 2",
  "term_id": "GO:0033387"
}